{
  "gene": "UniProtKB:O75791",
  "gene_name": "GRB2-related adapter protein 2",
  "term_label": "regulation of MAPK cascade",
  "term_id": "GO:0043408",
  "gene_symbol": "GRAP2"
}